{
  "term_id": "UNKNOWN:0002",
  "gene_name": "Fanconi anemia core complex-associated protein 100",
  "term_label": "Unknown biological process",
  "gene_symbol": "FAAP100",
  "gene": "UniProtKB:Q0VG06"
}